regulation of cilium beat frequency [GO:0003356] (biological process) Sources: GOC:dph Note: Note that we deem cilium and microtubule-based flagellum to be equivalent. Subtypes: regulation of cilium beat frequency involved in ciliary motility [GO:0060296] Also known as: regulation of microtubule-based flagellum beat frequency, regulation of flagellum beat frequency Relationships: is a type of regulation of cilium movement [GO:0003352] Definition: Any process that modulates the frequency of cilium movement, the directed, self-propelled movement of a cilium.